{
  "gene_name": "Cathepsin E",
  "term_label": "endosome",
  "gene_symbol": "CTSE",
  "gene": "UniProtKB:P14091",
  "term_id": "GO:0005768"
}